{
  "gene_symbol": "DSCAM",
  "term_id": "GO:0007156",
  "term_label": "homophilic cell-cell adhesion",
  "gene_name": "Cell adhesion molecule DSCAM",
  "gene": "UniProtKB:O60469"
}